{
  "term_label": "chromatin",
  "term_id": "GO:0000785",
  "gene_symbol": "PIAS4",
  "gene": "UniProtKB:Q8N2W9",
  "gene_name": "E3 SUMO-protein ligase PIAS4"
}